{
  "gene_name": "Interleukin-37",
  "term_id": "GO:0006955",
  "gene": "UniProtKB:Q9NZH6",
  "gene_symbol": "IL37",
  "term_label": "immune response"
}